{
  "gene_symbol": "CCT2",
  "term_label": "unfolded protein binding",
  "term_id": "GO:0051082",
  "gene": "UniProtKB:P78371",
  "gene_name": "T-complex protein 1 subunit beta"
}